{
  "gene_symbol": "ITGAD",
  "term_label": "signaling receptor activity",
  "term_id": "GO:0038023",
  "gene_name": "Integrin alpha-D",
  "gene": "UniProtKB:Q13349"
}